caudal fin morphogenesis [GO:0035143] (biological process) Relationships: is a type of medial fin morphogenesis [GO:0035141]; BFO_0000050 caudal fin development [GO:0033336] Sources: GOC:dgh Definition: The process in which the anatomical structures of the caudal fin are generated and organized. A caudal fin is an unpaired medial fin mounted at the caudal end of the fish, and is the main fin used for propulsion. Subtypes: GO:0035124, post-embryonic caudal fin morphogenesis [GO:0035133]